{
  "gene_symbol": "PARP4",
  "gene_name": "Protein mono-ADP-ribosyltransferase PARP4",
  "term_id": "GO:0005737",
  "term_label": "cytoplasm",
  "gene": "UniProtKB:Q9UKK3"
}